protein-phosphocysteine-glucosamine phosphotransferase system transporter activity [GO:0090587] (molecular function) Definition: Catalysis of the PEP-dependent, phosphoryl transfer-driven transport of substances across a membrane. The transport happens by catalysis of the reaction: protein S-phosphocysteine + glucosamine (out) = protein cysteine + glucosamine-6-phosphate (in). References: PMID:8246840 Relationships: is a type of GO:0090563